pterin deaminase activity [GO:0050228] (molecular function) Relationships: is a type of hydrolase activity, acting on carbon-nitrogen (but not peptide) bonds, in cyclic amidines [GO:0016814]; is a type of GO:0019239 Also known as: 2-amino-4-hydroxypteridine aminohydrolase activity, acrasinase activity Sources: RHEA:36055 Definition: Catalysis of the reaction: a 2-amino-4-hydroxypteridine + H2O + H+ = a 2,4-dihydroxypteridine + NH4+.